{
  "term_label": "mitochondrion organization",
  "term_id": "GO:0007005",
  "gene_name": "Pentatricopeptide repeat-containing protein 2, mitochondrial",
  "gene_symbol": "PTCD2",
  "gene": "UniProtKB:Q8WV60"
}